{
  "term_id": "UNKNOWN:0001",
  "gene_name": "Transmembrane protein 18",
  "gene": "UniProtKB:Q96B42",
  "term_label": "Unknown molecular function",
  "gene_symbol": "TMEM18"
}